{
  "gene": "UniProtKB:A8MTA8",
  "term_label": "Unknown biological process",
  "term_id": "UNKNOWN:0002",
  "gene_symbol": "FAM166B",
  "gene_name": "Protein FAM166B"
}